cellular stress response to acidic pH [GO:1990451] (biological process) References: PMID:10615049 Sources: GOC:BHF, GOC:go_curators, GOC:rl Definition: Any process that results in a change in state or activity of a cell (in terms of movement, secretion, enzyme production, gene expression, etc.) as a result of a disturbance in the homeostasis of organismal or cellular pH (with pH < 7). pH is a measure of the acidity or basicity of an aqueous solution. Relationships: is a type of cellular response to chemical stress [GO:0062197]; is a type of cellular response to acidic pH [GO:0071468] Note: An example of this is NOX1 in human (Q9Y5S8) in PMID:10615049. Also known as: cellular stress response to acidity